{
  "term_label": "Unknown biological process",
  "gene_symbol": "GOLT1A",
  "term_id": "UNKNOWN:0002",
  "gene": "UniProtKB:Q6ZVE7",
  "gene_name": "Vesicle transport protein GOT1A"
}